type-II cohesin domain binding [GO:1990312] (molecular function) Relationships: is_a protein domain specific binding [GO:0019904] References: PMID:23195689, PMID:24080387 Sources: GOC:mengo_curators Definition: Binding to a type-II cohesin domain of a protein. Type-II cohesin domain is the binding partner of type-II dockerin domain.